{
  "term_label": "insulin receptor complex",
  "gene_name": "Insulin-like growth factor 1 receptor",
  "term_id": "GO:0005899",
  "gene": "UniProtKB:P08069",
  "gene_symbol": "IGF1R"
}